{
  "gene_name": "Glucagon receptor",
  "term_label": "peptide hormone binding",
  "term_id": "GO:0017046",
  "gene_symbol": "GCGR",
  "gene": "UniProtKB:P47871"
}